{
  "gene": "UniProtKB:Q9GZN0",
  "term_label": "cellular response to light stimulus",
  "gene_symbol": "GPR88",
  "gene_name": "Probable G-protein coupled receptor 88",
  "term_id": "GO:0071482"
}